proboscis extension reflex [GO:0007637] (BP) Relationships: is a type of chemosensory behavior [GO:0007635]; is a type of behavioral response to nutrient [GO:0051780]; is a type of reflex [GO:0060004] Sources: FB:FBrf0044924, GOC:jid Definition: The extension, through direct muscle actions, of the proboscis (the trunk-like extension of the mouthparts on the adult external head) in response to a nutritional stimulus. Also known as: behavioral response to nutritional stimulus, proboscis extension, proboscis extension in response to nutritional stimulus